hypochlorite binding [GO:1901531] (molecular function) References: PMID:22223481 Sources: GOC:TermGenie, GOC:pr Definition: Binding to hypochlorite. Relationships: is a type of anion binding [GO:0043168]